{
  "term_id": "GO:0007186",
  "gene_name": "Adhesion G protein-coupled receptor L2",
  "gene": "UniProtKB:O95490",
  "gene_symbol": "ADGRL2",
  "term_label": "G protein-coupled receptor signaling pathway"
}